{
  "gene_name": "Sec1 family domain-containing protein 1",
  "term_id": "GO:0019905",
  "gene": "UniProtKB:Q8WVM8",
  "gene_symbol": "SCFD1",
  "term_label": "syntaxin binding"
}